{
  "term_label": "Unknown molecular function",
  "gene_symbol": "ZSWIM9",
  "gene_name": "Uncharacterized protein ZSWIM9",
  "term_id": "UNKNOWN:0001",
  "gene": "UniProtKB:Q86XI8"
}